serine binding [GO:0070905] (molecular function) Relationships: is a type of amino acid binding [GO:0016597]; is a type of carboxylic acid binding [GO:0031406]; is a type of cation binding [GO:0043169] Definition: Binding to 2-amino-3-hydroxypropanoic acid. Also known as: Ser binding Sources: GOC:rph